negative regulation of o-orsellinic acid biosynthetic process [GO:1900699] (BP) Definition: Any process that stops, prevents or reduces the frequency, rate or extent of o-orsellinic acid biosynthetic process. Sources: GOC:TermGenie, GOC:di Also known as: down regulation of o-orsellinic acid anabolism, down regulation of o-orsellinic acid biosynthesis, down regulation of o-orsellinic acid biosynthetic process, down regulation of o-orsellinic acid formation, down regulation of o-orsellinic acid synthesis, down-regulation of o-orsellinic acid anabolism, down-regulation of o-orsellinic acid biosynthesis, down-regulation of o-orsellinic acid biosynthetic process, down-regulation of o-orsellinic acid formation, down-regulation of o-orsellinic acid synthesis, downregulation of o-orsellinic acid anabolism, downregulation of o-orsellinic acid biosynthesis, downregulation of o-orsellinic acid biosynthetic process, downregulation of o-orsellinic acid formation, downregulation of o-orsellinic acid synthesis, inhibition of o-orsellinic acid anabolism, inhibition of o-orsellinic acid biosynthesis, inhibition of o-orsellinic acid formation, inhibition of o-orsellinic acid synthesis, negative regulation of o-orsellinic acid anabolism, negative regulation of o-orsellinic acid biosynthesis, negative regulation of o-orsellinic acid formation, negative regulation of o-orsellinic acid synthesis, inhibition of o-orsellinic acid biosynthetic process Relationships: is a type of negative regulation of small molecule metabolic process [GO:0062014]; is a type of negative regulation of secondary metabolite biosynthetic process [GO:1900377]; is a type of regulation of o-orsellinic acid biosynthetic process [GO:1900698]; RO_0002212 o-orsellinic acid biosynthetic process [GO:1900584]